{
  "term_label": "microtubule motor activity",
  "gene_name": "Kinesin-like protein KIF25",
  "gene": "UniProtKB:Q9UIL4",
  "term_id": "GO:0003777",
  "gene_symbol": "KIF25"
}